{
  "term_label": "COPII-coated ER to Golgi transport vesicle",
  "gene": "UniProtKB:Q5BJH7",
  "term_id": "GO:0030134",
  "gene_symbol": "YIF1B",
  "gene_name": "Protein YIF1B"
}